{
  "gene": "UniProtKB:P07237",
  "term_id": "GO:0006457",
  "gene_name": "Protein disulfide-isomerase",
  "term_label": "protein folding",
  "gene_symbol": "P4HB"
}